granulocyte migration [GO:0097530] (biological process) Definition: The movement of a granulocyte within or between different tissues and organs of the body. Subtypes: granulocyte chemotaxis [GO:0071621], eosinophil migration [GO:0072677], neutrophil migration [GO:1990266] References: PMID:24163421, PMID:24193336 Sources: GOC:cvs Relationships: is a type of myeloid leukocyte migration [GO:0097529]